{
  "gene_symbol": "RPS9",
  "gene": "UniProtKB:P46781",
  "term_label": "structural constituent of ribosome",
  "term_id": "GO:0003735",
  "gene_name": "Small ribosomal subunit protein uS4"
}